{
  "term_id": "GO:0016538",
  "gene_name": "G2_mitotic-specific cyclin-B2",
  "gene": "UniProtKB:O95067",
  "gene_symbol": "CCNB2",
  "term_label": "cyclin-dependent protein serine/threonine kinase regulator activity"
}